{
  "term_id": "GO:0009897",
  "gene_symbol": "HLA-G",
  "gene": "UniProtKB:P17693",
  "gene_name": "HLA class I histocompatibility antigen, alpha chain G",
  "term_label": "external side of plasma membrane"
}